{
  "gene_symbol": "ACSM3",
  "gene": "UniProtKB:Q53FZ2",
  "term_label": "fatty acid biosynthetic process",
  "gene_name": "Acyl-coenzyme A synthetase ACSM3, mitochondrial",
  "term_id": "GO:0006633"
}